chromosome, telomeric region [GO:0000781] (cellular component) Note: Note that this term can be used in place of the obsolete cellular component term 'telomere ; GO:0005696'. Use with caution because this term refers to a specific region of the chromosome and not a protein complex. Subtypes: chromosome, subtelomeric region [GO:0099115], chromosome, telomeric repeat region [GO:0140445] Also known as: nuclear chromosome, telomere, nuclear chromosome, telomeric region, telomere Definition: The end of a linear chromosome, required for the integrity and maintenance of the end. A chromosome telomere usually includes a region of telomerase-encoded repeats the length of which rarely exceeds 20 bp each and that permits the formation of a telomeric loop (T-loop). The telomeric repeat region is usually preceded by a sub-telomeric region that is gene-poor but rich in repetitive elements. Some telomeres only consist of the latter part (for eg. D. melanogaster telomeres). Sources: GOC:elh Relationships: is a type of chromosomal region [GO:0098687]